{
  "gene": "UniProtKB:P80075",
  "gene_symbol": "CCL8",
  "term_id": "GO:0030335",
  "term_label": "positive regulation of cell migration",
  "gene_name": "C-C motif chemokine 8"
}